lipopolysaccharide immune receptor activity [GO:0001875] (molecular function) Relationships: is a type of pattern recognition receptor activity [GO:0038187]; is part of lipopolysaccharide-mediated signaling pathway [GO:0031663]; has part lipopolysaccharide binding [GO:0001530] Definition: Combining with a lipopolysaccharide and transmitting the signal across the cell membrane to initiate an innate immune response. Lipopolysaccharides (LPS) are major components of the outer membrane of Gram-negative bacteria, making them prime targets for recognition by the immune system. References: PMID:14609719, PMID:15379975 Also known as: endotoxin receptor activity, lipopolysaccharide receptor activity, LPS receptor activity